pore complex [GO:0046930] (cellular component) Also known as: pore, channel-forming toxin activity, pore-forming toxin activity Relationships: is a type of GO:0098796 Definition: A protein complex providing a discrete opening in a membrane that allows the passage of gases and/or liquids. Sources: ISBN:0198506732 Subtypes: membrane attack complex [GO:0005579], GO:0005757, glomerular endothelium fenestra [GO:0036053]